{
  "term_id": "UNKNOWN:0002",
  "term_label": "Unknown biological process",
  "gene_symbol": "IMPG2",
  "gene": "UniProtKB:Q9BZV3",
  "gene_name": "Interphotoreceptor matrix proteoglycan 2"
}